{
  "term_id": "GO:0006955",
  "gene_name": "T cell receptor alpha variable 38-2_delta variable 8",
  "term_label": "immune response",
  "gene_symbol": "TRAV38-2DV8",
  "gene": "UniProtKB:A0JD32"
}